{
  "term_id": "GO:0043113",
  "gene_symbol": "DLG2",
  "gene": "UniProtKB:Q15700",
  "term_label": "receptor clustering",
  "gene_name": "Disks large homolog 2"
}